venom-mediated suppression of blood coagulation [GO:0044470] (biological process) Sources: GOC:jl Also known as: envenomation resulting in negative regulation of blood coagulation in another organism, envenomation resulting in negative regulation of blood coagulation in other organism, envenomation suppressing blood coagulation Relationships: is a type of venom-mediated perturbation of blood coagulation [GO:0044468] Definition: A process in which an organism inhibits or disrupts blood coagulation in another organism via the action of a venom.